baroreceptor detection of arterial stretch [GO:0001981] (biological process) Relationships: is a type of vascular process in circulatory system [GO:0003018]; is a type of detection of mechanical stimulus [GO:0050982]; is part of regulation of systemic arterial blood pressure by carotid sinus baroreceptor feedback [GO:0001978] Definition: The series of events by which the change in diameter of an artery is detected and converted to a molecular signal. Subtypes: baroreceptor detection of increased arterial stretch [GO:0003023], baroreceptor detection of decreased arterial stretch [GO:0003024] Sources: GOC:mtg_cardio, ISBN:0721643949